{
  "gene_name": "Protein NDRG4",
  "gene": "UniProtKB:Q9ULP0",
  "gene_symbol": "NDRG4",
  "term_label": "cytoplasm",
  "term_id": "GO:0005737"
}